{
  "gene": "UniProtKB:Q9BX97",
  "term_id": "UNKNOWN:0001",
  "gene_name": "Plasmalemma vesicle-associated protein",
  "term_label": "Unknown molecular function",
  "gene_symbol": "PLVAP"
}